double-stranded RNA-specific ribonuclease activity [GO:0032296] (molecular function) Subtypes: ribonuclease III activity [GO:0004525] Relationships: is a type of GO:0004540; is a type of GO:0016788 Also known as: double-stranded RNA-specific RNase activity, dsRNA-specific RNase activity, dsRNA-specific ribonuclease activity Sources: GOC:mah Definition: Catalysis of the hydrolysis of phosphodiester bonds in double-stranded RNA molecules.